{
  "gene_name": "Alpha-2-macroglobulin receptor-associated protein",
  "gene_symbol": "LRPAP1",
  "term_label": "endosome",
  "gene": "UniProtKB:P30533",
  "term_id": "GO:0005768"
}